{
  "gene": "UniProtKB:P54257",
  "gene_name": "Huntingtin-associated protein 1",
  "term_label": "protein targeting",
  "gene_symbol": "HAP1",
  "term_id": "GO:0006605"
}